{
  "gene_symbol": "SLC9A7",
  "term_label": "recycling endosome",
  "gene": "UniProtKB:Q96T83",
  "gene_name": "Sodium_hydrogen exchanger 7",
  "term_id": "GO:0055037"
}